{
  "gene_symbol": "RC3H2",
  "gene_name": "Roquin-2",
  "term_label": "cytoplasmic stress granule",
  "term_id": "GO:0010494",
  "gene": "UniProtKB:Q9HBD1"
}